{
  "gene_name": "Hippocampus abundant transcript-like protein 1",
  "term_label": "Unknown biological process",
  "gene_symbol": "MFSD14B",
  "gene": "UniProtKB:Q5SR56",
  "term_id": "UNKNOWN:0002"
}